{
  "gene_name": "WD repeat domain phosphoinositide-interacting protein 3",
  "term_id": "GO:0034497",
  "gene_symbol": "WDR45B",
  "gene": "UniProtKB:Q5MNZ6",
  "term_label": "protein localization to phagophore assembly site"
}